presynaptic intermediate filament cytoskeleton [GO:0099182] (CC) Relationships: is a type of GO:0045111; is a type of presynaptic cytoskeleton [GO:0099569] Definition: The intermediate filament cytoskeleton that is part of a presynapse. Sources: GOC:dos